{
  "gene_name": "D-glutamate cyclase, mitochondrial",
  "term_id": "UNKNOWN:0003",
  "gene": "UniProtKB:Q7Z3D6",
  "gene_symbol": "DGLUCY",
  "term_label": "Unknown cellular component"
}